{
  "gene_name": "RNA-binding protein Musashi homolog 2",
  "gene_symbol": "MSI2",
  "term_label": "regulation of translation",
  "gene": "UniProtKB:Q96DH6",
  "term_id": "GO:0006417"
}